3'-5' DNA/RNA helicase activity [GO:0033679] (molecular function) Sources: GOC:mah Definition: Unwinding of a DNA/RNA duplex in the 3' to 5' direction, driven by ATP hydrolysis. Relationships: is a type of GO:0033677 Also known as: 3' to 5' DNA/RNA helicase activity, ATP-dependent 3' to 5' DNA/RNA helicase activity, ATP-dependent 3'-5' DNA/RNA helicase activity